{
  "gene": "UniProtKB:Q9HCU5",
  "gene_symbol": "PREB",
  "term_label": "Unknown molecular function",
  "term_id": "UNKNOWN:0001",
  "gene_name": "Prolactin regulatory element-binding protein"
}